{
  "gene_symbol": "SORT1",
  "term_id": "GO:0006897",
  "gene": "UniProtKB:Q99523",
  "gene_name": "Sortilin",
  "term_label": "endocytosis"
}